{
  "gene_symbol": "ARIH1",
  "term_id": "GO:0061630",
  "term_label": "ubiquitin protein ligase activity",
  "gene": "UniProtKB:Q9Y4X5",
  "gene_name": "E3 ubiquitin-protein ligase ARIH1"
}